{
  "term_label": "peptide antigen assembly with MHC class II protein complex",
  "gene_name": "Beta-2-microglobulin",
  "term_id": "GO:0002503",
  "gene_symbol": "B2M",
  "gene": "UniProtKB:P61769"
}